{
  "gene_symbol": "PGAM4",
  "term_id": "UNKNOWN:0002",
  "gene_name": "Probable phosphoglycerate mutase 4",
  "term_label": "Unknown biological process",
  "gene": "UniProtKB:Q8N0Y7"
}